D-ribose 5-phosphate biosynthetic process [GO:1901280] (BP) Also known as: D-ribose 5-phosphate anabolism, D-ribose 5-phosphate biosynthesis, D-ribose 5-phosphate formation, D-ribose 5-phosphate synthesis Definition: The chemical reactions and pathways resulting in the formation of D-ribose 5-phosphate. Sources: GOC:TermGenie, GOC:yaf, UniPathway:UPA00293 Relationships: is a type of ribose phosphate biosynthetic process [GO:0046390]